{
  "term_label": "Unknown molecular function",
  "gene_symbol": "CEACAM8",
  "gene": "UniProtKB:P31997",
  "term_id": "UNKNOWN:0001",
  "gene_name": "Carcinoembryonic antigen-related cell adhesion molecule 8"
}